{
  "gene": "UniProtKB:O14980",
  "gene_name": "Exportin-1",
  "term_label": "ribosomal large subunit export from nucleus",
  "term_id": "GO:0000055",
  "gene_symbol": "XPO1"
}